alpha-amino-acid esterase activity [GO:0047658] (molecular function) Relationships: is a type of carboxylic ester hydrolase activity [GO:0052689] Sources: EC:3.1.1.43, MetaCyc:ALPHA-AMINO-ACID-ESTERASE-RXN Definition: Catalysis of the reaction: an alpha-amino acid ester + H2O = an alpha-amino acid + an alcohol. Also known as: a-amino-acid esterase activity, alpha-amino acid ester hydrolase activity, alpha-amino-acid ester hydrolase activity, alpha-amino-acid-ester aminoacylhydrolase activity